{
  "gene": "UniProtKB:P49356",
  "gene_symbol": "FNTB",
  "term_label": "protein farnesyltransferase activity",
  "gene_name": "Protein farnesyltransferase subunit beta",
  "term_id": "GO:0004660"
}